{
  "term_id": "GO:0046427",
  "gene_symbol": "LEP",
  "gene": "UniProtKB:P41159",
  "term_label": "positive regulation of receptor signaling pathway via JAK-STAT",
  "gene_name": "Leptin"
}